{
  "gene": "UniProtKB:Q96CW1",
  "gene_name": "AP-2 complex subunit mu",
  "term_id": "GO:0005829",
  "term_label": "cytosol",
  "gene_symbol": "AP2M1"
}